beta-alanine catabolic process [GO:0019484] (biological process) Definition: The chemical reactions and pathways resulting in the breakdown of beta-alanine (3-aminopropanoic acid), an achiral amino acid and an isomer of alanine. It occurs free (e.g. in brain) and in combination (e.g. in pantothenate) but it is not a constituent of proteins. Sources: GOC:jl, ISBN:0198506732 Also known as: beta-alanine breakdown, beta-alanine catabolism, beta-alanine degradation Relationships: is a type of amino acid catabolic process [GO:0009063]; is a type of beta-alanine metabolic process [GO:0019482]; is a type of GO:0170044 Subtypes: beta-alanine catabolic process to L-alanine [GO:0019485], GO:0019486